{
  "term_label": "late endosome membrane",
  "term_id": "GO:0031902",
  "gene": "UniProtKB:P01906",
  "gene_symbol": "HLA-DQA2",
  "gene_name": "HLA class II histocompatibility antigen, DQ alpha 2 chain"
}